{
  "gene": "UniProtKB:E9PGG2",
  "term_id": "GO:0005667",
  "gene_name": "Anomalous homeobox protein",
  "term_label": "transcription regulator complex",
  "gene_symbol": "ANHX"
}